{
  "term_label": "intraciliary transport",
  "gene_name": "Lebercilin-like protein",
  "term_id": "GO:0042073",
  "gene": "UniProtKB:O95447",
  "gene_symbol": "LCA5L"
}